luteinizing hormone receptor activity [GO:0004964] (molecular function) Definition: Combining with luteinizing hormone (also called lutropin) to initiate a change in cell activity. Relationships: is a type of GO:0004930; is a type of GO:0016500; BFO_0000050 luteinizing hormone signaling pathway [GO:0042700] Also known as: LH receptor, LHR, lutropin receptor, lutropin-choriogonadotropic hormone receptor References: PMID:18848524, PMID:1922095 Sources: ISBN:0198506732